cellular response to toxic substance [GO:0097237] (biological process) Relationships: is_a response to toxic substance [GO:0009636]; is a type of cellular response to chemical stimulus [GO:0070887] Subtypes: cellular response to mycotoxin [GO:0036146] Definition: Any process that results in a change in state or activity of a cell (in terms of movement, secretion, enzyme production, gene expression, etc.) as a result of a toxic stimulus. Sources: GOC:pr